metanephric mesenchyme morphogenesis [GO:0072133] (biological process) Sources: GOC:mtg_kidney_jan10 Relationships: is a type of kidney mesenchyme morphogenesis [GO:0072131]; is part of metanephric mesenchyme development [GO:0072075] Subtypes: metanephric cap morphogenesis [GO:0072186] Definition: The process in which the anatomical structures of a metanephric mesenchymal tissue are generated and organized. Metanephric mesenchyme is the tissue made up of loosely connected mesenchymal cells in the metanephros.